blood vessel diameter maintenance [GO:0097746] (BP) Relationships: is a type of GO:0003018; is a type of regulation of tube diameter [GO:0035296]; is part of blood circulation [GO:0008015] Sources: GOC:pr Subtypes: maintenance of blood vessel diameter homeostasis by renin-angiotensin [GO:0002034], GO:0019229, vasoconstriction [GO:0042310], vasodilation [GO:0042311] Definition: Any process that modulates the diameter of blood vessels. Also known as: blood vessel diameter homeostasis, regulation of blood vessel diameter, regulation of blood vessel size, regulation of vasodilatation, regulation of vasodilation